{
  "gene": "UniProtKB:P28070",
  "gene_name": "Proteasome subunit beta type-4",
  "gene_symbol": "PSMB4",
  "term_id": "GO:0043161",
  "term_label": "proteasome-mediated ubiquitin-dependent protein catabolic process"
}